histone H2AT120pho reader activity [GO:0140172] (molecular function) Relationships: is a type of histone H2A reader activity [GO:0140054] Definition: A histone reader that recognizes a histone H2A phosphorylated at threonine 120. References: PMID:19965387, PMID:20679485 Note: Note that the residue position corresponds to the canonical human H2A2A histone (UniProtKB:Q6FI13); this residue is conserved across all eukaryotes, but corresponds to T119 in Drosophila and S121 in yeast and Tetrahymena. Residue 1 is the first residue following removal of the initiating Methionine (Met). Note that each histone is encoded by multiple genes, and sequences may vary across different genes within an organism. Also known as: histone H2AS120pho reader activity